L-arabinose catabolic process to 2-oxoglutarate [GO:0019570] (biological process) Sources: GOC:go_curators Relationships: is a type of 2-oxoglutarate metabolic process [GO:0006103]; is_a GO:0019572 Definition: The chemical reactions and pathways resulting in the breakdown of L-arabinose into other compounds, including 2-oxoglutarate. Also known as: L-arabinose breakdown to 2-oxoglutarate, L-arabinose catabolic process to 2-ketoglutarate, L-arabinose catabolic process to alpha-ketoglutarate, L-arabinose catabolic process to alpha-oxoglutarate, L-arabinose catabolism to 2-ketoglutarate, L-arabinose catabolism to alpha-ketoglutarate, L-arabinose catabolism to alpha-oxoglutarate, L-arabinose degradation to 2-oxoglutarate